{
  "gene_symbol": "PIEZO1",
  "term_id": "GO:0071260",
  "gene_name": "Piezo-type mechanosensitive ion channel component 1",
  "gene": "UniProtKB:Q92508",
  "term_label": "cellular response to mechanical stimulus"
}